transitional stage B cell differentiation [GO:0002332] (biological process) Relationships: is a type of immature B cell differentiation [GO:0002327] Definition: The process in which immature B cells from the bone marrow become mature B cells in the spleen. Transitional stage B cells are subdivided into transitional one (T1) and transitional two (T2) stages and are short-lived and functionally incompetent. Note: Note that immunologists typically use the word 'development' to refer to cells of B or T cell lineages undergoing the process that GO describes as 'cell differentiation'. Sources: GOC:jal, ISBN:0781735149 Subtypes: transitional one stage B cell differentiation [GO:0002333], transitional two stage B cell differentiation [GO:0002334] Also known as: transitional stage B lymphocyte differentiation, transitional stage B-cell differentiation, transitional stage B-lymphocyte differentiation, transitional stage B cell development